spermine oxidase activity [GO:0052901] (molecular function) Relationships: is a type of polyamine oxidase activity [GO:0046592] Definition: Catalysis of the reaction: H2O + O2 + spermine = 3-aminopropanal + H2O2 + spermidine. Weak activity with N(1)-acetylspermine. The Arabidopsis thaliana enzyme converts norspermine to norspermidine. Sources: EC:1.5.3.16, RHEA:25804 Also known as: spermine:oxygen oxidoreductase (spermidine-forming) activity